{
  "gene_symbol": "XPOT",
  "gene": "UniProtKB:O43592",
  "term_label": "tRNA re-export from nucleus",
  "term_id": "GO:0071528",
  "gene_name": "Exportin-T"
}